{
  "term_label": "extracellular space",
  "gene_name": "Tissue-type plasminogen activator",
  "gene": "UniProtKB:P00750",
  "gene_symbol": "PLAT",
  "term_id": "GO:0005615"
}